retinal isomerization [GO:0106434] (biological process) Relationships: is a type of retinal metabolic process [GO:0042574] References: PMID:21447403 Note: This process term replaces 'retinal isomerase' because the Enzyme Commission has determined that the reaction is known to be catalyzed by a pathway involving multiple steps, catalyzed by EC:1.1.1.300, EC:2.3.1.135, EC:3.1.1.64, and EC:1.1.1.315. Definition: The reactions involved in isomerization of all trans to all cis retnal.